negative regulation of establishment of competence for transformation [GO:0045808] (biological process) Definition: Any process that stops, prevents, or reduces the frequency, rate or extent of establishment of competence for transformation. Sources: GOC:go_curators Also known as: down regulation of establishment of competence for transformation, down-regulation of establishment of competence for transformation, downregulation of establishment of competence for transformation, inhibition of establishment of competence for transformation, inhibitor of the establishment of competence for transformation activity Relationships: is a type of GO:0045304; is a type of negative regulation of cellular process [GO:0048523]; is_a negative regulation of response to stimulus [GO:0048585]; negatively regulates establishment of competence for transformation [GO:0030420]